{
  "gene": "UniProtKB:Q6IC98",
  "gene_name": "GRAM domain-containing protein 4",
  "term_id": "GO:0005739",
  "gene_symbol": "GRAMD4",
  "term_label": "mitochondrion"
}